{
  "term_label": "ubiquitin protein ligase activity",
  "term_id": "GO:0061630",
  "gene_name": "E3 ubiquitin-protein ligase MARCHF6",
  "gene": "UniProtKB:O60337",
  "gene_symbol": "MARCHF6"
}